{
  "gene_name": "Oxysterols receptor LXR-alpha",
  "term_id": "GO:0004879",
  "term_label": "nuclear receptor activity",
  "gene_symbol": "NR1H3",
  "gene": "UniProtKB:Q13133"
}